{
  "term_id": "GO:0043652",
  "gene_name": "XK-related protein 4",
  "gene_symbol": "XKR4",
  "gene": "UniProtKB:Q5GH76",
  "term_label": "engulfment of apoptotic cell"
}